{
  "gene_symbol": "IL22",
  "term_id": "GO:0005125",
  "term_label": "cytokine activity",
  "gene_name": "Interleukin-22",
  "gene": "UniProtKB:Q9GZX6"
}